{
  "gene_name": "Nitric oxide-associated protein 1",
  "term_id": "UNKNOWN:0001",
  "gene_symbol": "NOA1",
  "term_label": "Unknown molecular function",
  "gene": "UniProtKB:Q8NC60"
}